{
  "term_id": "GO:0016477",
  "term_label": "cell migration",
  "gene": "UniProtKB:P55287",
  "gene_name": "Cadherin-11",
  "gene_symbol": "CDH11"
}